{
  "gene_symbol": "GSC",
  "gene": "UniProtKB:P56915",
  "term_label": "regulation of transcription by RNA polymerase II",
  "term_id": "GO:0006357",
  "gene_name": "Homeobox protein goosecoid"
}